regulation of postsynaptic dense core vesicle exocytosis [GO:0150044] (biological process) References: PMID:19448629 Sources: GOC:aruk, GOC:bc Relationships: is a type of regulation of dense core granule exocytosis [GO:1905413]; regulates postsynaptic dense core vesicle exocytosis [GO:0150038] Definition: Any process that modulates the frequency, rate or extent of postsynaptic dense core vesicle exocytosis.